{
  "term_id": "GO:0005634",
  "term_label": "nucleus",
  "gene_name": "Ubiquitin-conjugating enzyme E2 D1",
  "gene": "UniProtKB:P51668",
  "gene_symbol": "UBE2D1"
}